{
  "gene": "UniProtKB:Q9BZE7",
  "term_label": "Unknown molecular function",
  "term_id": "UNKNOWN:0001",
  "gene_name": "UPF0193 protein EVG1",
  "gene_symbol": "C22orf23"
}